slime layer polysaccharide biosynthetic process [GO:0045228] (biological process) Sources: GOC:go_curators Relationships: is a type of polysaccharide biosynthetic process [GO:0000271]; is a type of slime layer organization [GO:0045231] Also known as: slime layer polysaccharide anabolism, slime layer polysaccharide biosynthesis, slime layer polysaccharide formation, slime layer polysaccharide synthesis Definition: The chemical reactions and pathways resulting in the formation of polysaccharides in the slime layer, a diffused layer of polysaccharide exterior to the bacterial cell wall.